acetyl-CoA catabolic process [GO:0046356] (biological process) Subtypes: acetyl-CoA assimilation pathway [GO:0019681] Relationships: is a type of acetyl-CoA metabolic process [GO:0006084]; is a type of sulfur compound catabolic process [GO:0044273]; is a type of purine-containing compound catabolic process [GO:0072523]; is a type of nucleoside phosphate catabolic process [GO:1901292] Definition: The chemical reactions and pathways resulting in the breakdown of acetyl-CoA, a derivative of coenzyme A in which the sulfhydryl group is acetylated. Also known as: acetyl-CoA breakdown, acetyl-CoA catabolism, acetyl-CoA degradation Sources: GOC:ai